positive regulation of spore encystment on host [GO:0075216] (biological process) Subtypes: positive regulation of zoospore encystment on host [GO:0075220] Sources: GOC:pamgo_curators Definition: Any process that activates, maintains or increases the frequency, rate or extent of spore encystment on host. The host is defined as the larger of the organisms involved in a symbiotic interaction. Relationships: is_a positive regulation of cell development [GO:0010720]; is a type of modulation of spore encystment on host [GO:0075215]; positively regulates spore encystment [GO:0075214]